{
  "term_label": "detoxification of copper ion",
  "term_id": "GO:0010273",
  "gene_name": "Metallothionein-1B",
  "gene_symbol": "MT1B",
  "gene": "UniProtKB:P07438"
}